thiomorpholine-carboxylate dehydrogenase activity [GO:0047127] (molecular function) Definition: Catalysis of the reaction: NAD(P)+ + thiomorpholine-3-carboxylate = NAD(P)H + 3,4-dehydro-1,4-thiomorpholine-3-carboxylate. Relationships: is a type of oxidoreductase activity, acting on the CH-NH group of donors, NAD or NADP as acceptor [GO:0016646] Sources: EC:1.5.1.25, MetaCyc:1.5.1.25-RXN Also known as: ketimine reductase activity, ketimine-reducing enzyme, thiomorpholine-3-carboxylate:NAD(P)+ 5,6-oxidoreductase activity